regulation of glutamate secretion [GO:0014048] (biological process) Sources: GOC:ef Subtypes: positive regulation of glutamate secretion [GO:0014049], negative regulation of glutamate secretion [GO:0014050], regulation of glutamate secretion, neurotransmission [GO:1903294] Definition: Any process that modulates the frequency, rate or extent of the controlled release of glutamate. Relationships: is_a regulation of organic acid transport [GO:0032890]; is a type of regulation of amino acid transport [GO:0051955]; is a type of regulation of secretion by cell [GO:1903530]; regulates glutamate secretion [GO:0014047]